{
  "gene_name": "DNA repair protein RAD51 homolog 2",
  "gene": "UniProtKB:O15315",
  "term_id": "GO:0008094",
  "gene_symbol": "RAD51B",
  "term_label": "ATP-dependent activity, acting on DNA"
}